{
  "gene_name": "Testis-expressed protein 101",
  "term_label": "plasma membrane raft",
  "gene": "UniProtKB:Q9BY14",
  "term_id": "GO:0044853",
  "gene_symbol": "TEX101"
}